{
  "gene_symbol": "F2",
  "term_id": "GO:0030168",
  "term_label": "platelet activation",
  "gene": "UniProtKB:P00734",
  "gene_name": "Prothrombin"
}